regulation of helvolic acid biosynthetic process [GO:1900840] (biological process) Sources: GOC:TermGenie, GOC:di Definition: Any process that modulates the frequency, rate or extent of helvolic acid biosynthetic process. Relationships: is a type of regulation of ketone biosynthetic process [GO:0010566]; is a type of regulation of steroid biosynthetic process [GO:0050810]; is a type of regulation of secondary metabolite biosynthetic process [GO:1900376]; regulates helvolic acid biosynthetic process [GO:1900812] Subtypes: negative regulation of helvolic acid biosynthetic process [GO:1900841], positive regulation of helvolic acid biosynthetic process [GO:1900842]